{
  "term_id": "GO:0030148",
  "gene_symbol": "HACD4",
  "gene": "UniProtKB:Q5VWC8",
  "term_label": "sphingolipid biosynthetic process",
  "gene_name": "Very-long-chain (3R)-3-hydroxyacyl-CoA dehydratase 4"
}